histone H3R8 methyltransferase activity [GO:0140592] (MF) References: PMID:20708585, PMID:31533925 Definition: Catalysis of the reaction: S-adenosyl-L-methionine + (histone H3)-arginine (position 8) = S-adenosyl-L-homocysteine + (histone H3-N-methyl-arginine (position 8). This reaction is the addition of a methyl group to the arginine residue at position 8 of histone H3. Note: Comment: Note that the residue position corresponds to the canonical human H3 histone (UniProtKB:P84243); this residue is conserved across all eukaryotes. Residue 1 is the first residue following removal of the initiating Methionine (Met). Note that each histone is encoded by multiple genes, and sequences may vary across different genes within an organism. Also known as: histone H3R8 arginine methylase activity, histone H3R8 arginine methyltransferase activity, histone methyltransferase activity (H3-R8 specific), histone-H3R8 methyltransferase activity Relationships: is a type of protein-arginine N-methyltransferase activity [GO:0016274]; is a type of histone H3 methyltransferase activity [GO:0140938]